{
  "term_id": "GO:0016602",
  "term_label": "CCAAT-binding factor complex",
  "gene": "UniProtKB:Q13952",
  "gene_name": "Nuclear transcription factor Y subunit gamma",
  "gene_symbol": "NFYC"
}